{
  "gene": "UniProtKB:P33681",
  "gene_symbol": "CD80",
  "term_label": "T cell costimulation",
  "gene_name": "T-lymphocyte activation antigen CD80",
  "term_id": "GO:0031295"
}